{
  "term_id": "GO:0030864",
  "gene_name": "Alpha-actinin-1",
  "gene_symbol": "ACTN1",
  "term_label": "cortical actin cytoskeleton",
  "gene": "UniProtKB:P12814"
}